phosphoramidate-hexose phosphotransferase activity [GO:0047329] (molecular function) Also known as: phosphoramidate-hexose transphosphorylase activity, phosphoramidate:hexose 1-phosphotransferase activity, phosphoramidic-hexose transphosphorylase activity Sources: EC:2.7.1.62, MetaCyc:2.7.1.62-RXN Definition: Catalysis of the reaction: hexose + phosphoramidate = hexose 1-phosphate + NH3. Relationships: is a type of GO:0016301; is a type of phosphotransferase activity, alcohol group as acceptor [GO:0016773]